{
  "term_id": "GO:0005615",
  "gene": "UniProtKB:P16581",
  "term_label": "extracellular space",
  "gene_symbol": "SELE",
  "gene_name": "E-selectin"
}